B cell cytokine production [GO:0002368] (biological process) Sources: GOC:add, ISBN:0781735149 Regulation: regulated by regulation of B cell cytokine production [GO:0002721]; negatively regulated by negative regulation of B cell cytokine production [GO:0002722]; positively regulated by positive regulation of B cell cytokine production [GO:0002723] Relationships: is a type of cytokine production involved in immune response [GO:0002367]; is a type of B cell mediated immunity [GO:0019724] Definition: Any process that contributes to cytokine production by a B cell. Note: Note that this term is in the subset of terms that should not be used for direct gene product annotation. Instead, select one of the 'regulation' children terms. Also known as: B lymphocyte cytokine production, B-cell cytokine production, B-lymphocyte cytokine production